{
  "term_id": "GO:0004800",
  "gene_name": "Type I iodothyronine deiodinase",
  "gene": "UniProtKB:P49895",
  "term_label": "thyroxine 5'-deiodinase activity",
  "gene_symbol": "DIO1"
}